regulation of cell adhesion involved in growth plate cartilage morphogenesis [GO:0003436] (biological process) Sources: GOC:ascb_2009, GOC:dph, GOC:tb Definition: Any process that modulates the frequency, rate or extent of attachment of a cell to another cell or to the extracellular matrix and contributes to the shaping of the growth plate cartilage of an endochondral bone. Relationships: is a type of regulation of cell adhesion [GO:0030155]; is part of growth plate cartilage morphogenesis [GO:0003422]